{
  "gene": "UniProtKB:P51587",
  "term_label": "nucleus",
  "gene_name": "Breast cancer type 2 susceptibility protein",
  "gene_symbol": "BRCA2",
  "term_id": "GO:0005634"
}